{
  "gene_name": "Putative DBH-like monooxygenase protein 2",
  "gene": "UniProtKB:A6NHM9",
  "term_label": "octopamine biosynthetic process",
  "gene_symbol": "MOXD2P",
  "term_id": "GO:0006589"
}